{
  "term_id": "GO:0030036",
  "gene": "UniProtKB:Q8IY63",
  "term_label": "actin cytoskeleton organization",
  "gene_name": "Angiomotin-like protein 1",
  "gene_symbol": "AMOTL1"
}